{
  "term_label": "Unknown cellular component",
  "term_id": "UNKNOWN:0003",
  "gene_symbol": "ASTE1",
  "gene": "UniProtKB:Q2TB18",
  "gene_name": "Protein asteroid homolog 1"
}